negative regulation of extraocular skeletal muscle development [GO:0014726] (biological process) Relationships: is a type of regulation of extraocular skeletal muscle development [GO:0014725]; is a type of GO:0048642; negatively regulates extraocular skeletal muscle development [GO:0002074] Definition: Any process that stops, prevents, or reduces the frequency, rate or extent of extraocular skeletal muscle development. Extraocular skeletal muscle development is the process whose specific outcome is the progression of the extraocular skeletal muscle over time, from its formation to the mature structure. The extraocular muscle is derived from cranial mesoderm and controls eye movements. The muscle begins its development with the differentiation of the muscle cells and ends with the mature muscle. Sources: GOC:mtg_muscle